MAML3-RBP-Jkappa-ICN3 complex [GO:0071181] (cellular component) References: PMID:12370315 Definition: A protein complex that consists of the intracellular domain of Notch3 (ICN3), the DNA-binding transcription factor RBP-Jkappa, and the transcriptional coactivator Mastermind-like-3 (MAML3); the complex is involved in transcriptional activation in response to Notch-mediated signaling. Also known as: MAML3-RBP-Jkappa-Notch3 complex Relationships: is a type of nuclear protein-containing complex [GO:0140513]